nucleobase:monoatomic cation symporter activity [GO:0015391] (molecular function) Definition: Enables the transfer of a solute or solutes from one side of a membrane to the other according to the reaction: nucleobase(out) + cation(out) = nucleobase(in) + cation(in). Also known as: nucleobase:cation symporter activity Subtypes: GO:0015389, cytosine:proton symporter activity [GO:0015504], uracil:monoatomic cation symporter activity [GO:0015505] Sources: GOC:ai Relationships: is a type of nucleobase transmembrane transporter activity [GO:0015205]; is a type of solute:monoatomic cation symporter activity [GO:0015294]